{
  "term_label": "eukaryotic translation initiation factor 4F complex",
  "gene_name": "Eukaryotic translation initiation factor 4E",
  "gene_symbol": "EIF4E",
  "gene": "UniProtKB:P06730",
  "term_id": "GO:0016281"
}